cannabinoid receptor activity [GO:0004949] (MF) Sources: GOC:dph, IUPHAR_GPCR:1279, Wikipedia:Cannabinoid Relationships: is a type of GO:0004930; is part of GO:0038171 Also known as: cannaboid receptor, endocannabinoid receptor activity Definition: Combining with a cannabinoid to initiate a change in cell activity. Cannabinoids are a class of diverse chemical compounds that include the endocannabinoids and the phytocannabinoids.